{
  "gene": "UniProtKB:Q16613",
  "term_id": "GO:0007623",
  "gene_name": "Serotonin N-acetyltransferase",
  "term_label": "circadian rhythm",
  "gene_symbol": "AANAT"
}